RING-like zinc finger domain binding [GO:0071535] (molecular function) Definition: Binding to a RING-like zinc finger domain domain of a protein. The RING-like domain is a zinc finger domain that is related to the C3HC4 RING finger domain. Sources: GOC:mah, InterPro:IPR014857 Relationships: is a type of protein domain specific binding [GO:0019904]